protein-RNA complex organization [GO:0071826] (biological process) Also known as: RNA-protein complex subunit organization, protein-RNA complex subunit organization, ribonucleoprotein complex subunit organisation, ribonucleoprotein complex subunit organization Definition: Any process in which macromolecules aggregate, disaggregate, or are modified, resulting in the formation, disassembly, or alteration of a ribonucleoprotein complex. Relationships: is a type of protein-containing complex organization [GO:0043933] Sources: GOC:mah Subtypes: GO:0022618, protein-RNA complex disassembly [GO:0032988], protein-RNA complex remodeling [GO:0110136]